positive regulation of synapse maturation by synaptic transmission [GO:0090127] (biological process) Definition: Any process that increases the extent of synaptic maturation as a result of the communication from a pre-synaptic cell to a post-synaptic cell across a synapse. Sources: GOC:ascb_2009, GOC:dph, GOC:tb Relationships: is a type of chemical synaptic transmission [GO:0007268]; is a type of positive regulation of synapse maturation [GO:0090129]